axonal dopamine secretion [GO:0099124] (biological process) Also known as: axonal DA release, axonal dopamine release Relationships: is a type of dopamine secretion [GO:0014046]; is a type of establishment of localization in cell [GO:0051649]; occurs in axon [GO:0030424] References: PMID:21576241 Sources: GOC:PARL, GOC:bf Subtypes: dopamine secretion, neurotransmission [GO:0061527] Definition: The regulated release of dopamine from an axon.